{
  "gene_symbol": "PPARD",
  "term_label": "fatty acid metabolic process",
  "term_id": "GO:0006631",
  "gene_name": "Peroxisome proliferator-activated receptor delta",
  "gene": "UniProtKB:Q03181"
}